tRNA 2'-O-ribose methylation guide activity [GO:0030564] (molecular function) Definition: Specifies the site of 2'-O-ribose methylation in a tRNA molecule by base pairing with a short sequence around the target residue. Relationships: is a type of tRNA modification guide activity [GO:0030557]; is a type of RNA 2'-O-ribose methylation guide activity [GO:0030561] References: PMID:12457565 Sources: GOC:mah Note: Note that this term describes the activity of a nucleic acid, usually RNA, gene product that interacts with other RNA molecules via base pairing; it should not be used to annotate proteins.